{
  "term_label": "adenylate cyclase-modulating G protein-coupled receptor signaling pathway",
  "term_id": "GO:0007188",
  "gene": "UniProtKB:P08754",
  "gene_name": "Guanine nucleotide-binding protein G(i) subunit alpha-3",
  "gene_symbol": "GNAI3"
}